uropod retraction [GO:0034461] (biological process) Definition: The process in which a uropod detaches from the cell substrate and retracts the rear of a migrating cell. Relationships: is a type of uropod organization [GO:0032796] References: PMID:10704379 Sources: GOC:mah